protein-N(PI)-phosphohistidine-N,N'-diacetylchitobiose phosphotransferase system transporter activity [GO:0090562] (molecular function) Definition: Catalysis of the PEP-dependent, phosphoryl transfer-driven transport of substances across a membrane. The transport happens by catalysis of the reaction: protein N-phosphohistidine + N,N'-diacetylchitobiose(out) = protein histidine + N,N'-diacetylchitobiose phosphate(in). Relationships: is_a protein-N(PI)-phosphohistidine-sugar phosphotransferase activity [GO:0008982] References: PMID:10913119 Sources: GOC:am